positive regulation of T cell migration [GO:2000406] (biological process) Relationships: is_a positive regulation of lymphocyte migration [GO:2000403]; is a type of regulation of T cell migration [GO:2000404]; positively regulates T cell migration [GO:0072678] Also known as: positive regulation of T lymphocyte migration, positive regulation of T-cell migration, positive regulation of T-lymphocyte migration Definition: Any process that activates or increases the frequency, rate or extent of T cell migration. Subtypes: positive regulation of T cell chemotaxis [GO:0010820], GO:2000409, positive regulation of thymocyte migration [GO:2000412] Sources: GOC:mah